{
  "term_id": "GO:0090026",
  "gene_name": "C-X-C motif chemokine 17",
  "gene": "UniProtKB:Q6UXB2",
  "gene_symbol": "CXCL17",
  "term_label": "positive regulation of monocyte chemotaxis"
}